follicle-stimulating hormone activity [GO:0016913] (molecular function) Relationships: is a type of GO:0005179 Sources: ISBN:0198547684 Definition: The action characteristic of follicle-stimulating hormone (FSH), a gonadotrophic glycoprotein hormone secreted, in mammals, by the anterior pituitary gland. Upon receptor binding, FSH stimulates growth of Graafian follicles in the ovaries in females, and stimulates the epithelium of the seminiferous tubules to increase spermatogenesis. Also known as: FSH activity, follicle stimulating hormone activity, follitropin activity